{
  "gene_name": "DNA dC-dU-editing enzyme APOBEC-3G",
  "term_label": "nucleus",
  "term_id": "GO:0005634",
  "gene": "UniProtKB:Q9HC16",
  "gene_symbol": "APOBEC3G"
}